{
  "gene": "UniProtKB:Q9UBP0",
  "gene_symbol": "SPAST",
  "term_id": "GO:0051013",
  "gene_name": "Spastin",
  "term_label": "microtubule severing"
}